isopropylmalate transmembrane transporter activity [GO:0034658] (molecular function) Definition: Enables the transfer of isopropylmalate from one side of a membrane to the other. Sources: GOC:mah Relationships: is a type of GO:0005310; is part of isopropylmalate transport [GO:0034659]